regulation of protein acetylation [GO:1901983] (biological process) Definition: Any process that modulates the frequency, rate or extent of protein acetylation. Also known as: regulation of protein amino acid acetylation References: PMID:22117195 Sources: GOC:TermGenie Relationships: is a type of regulation of protein modification process [GO:0031399]; regulates GO:0006473 Subtypes: negative regulation of protein acetylation [GO:1901984], positive regulation of protein acetylation [GO:1901985], regulation of N-terminal peptidyl-methionine acetylation [GO:1904663], regulation of peptidyl-lysine acetylation [GO:2000756]